{
  "term_label": "RNA-3'-phosphate cyclase activity",
  "term_id": "GO:0003963",
  "gene": "UniProtKB:O00442",
  "gene_name": "RNA 3'-terminal phosphate cyclase",
  "gene_symbol": "RTCA"
}